{
  "term_label": "intermediate filament organization",
  "gene": "UniProtKB:Q6A162",
  "term_id": "GO:0045109",
  "gene_name": "Keratin, type I cytoskeletal 40",
  "gene_symbol": "KRT40"
}